{
  "gene_symbol": "HLA-DPB1",
  "term_label": "antigen processing and presentation of exogenous peptide antigen via MHC class II",
  "gene": "UniProtKB:P04440",
  "term_id": "GO:0019886",
  "gene_name": "HLA class II histocompatibility antigen, DP beta 1 chain"
}